ferric triacetylfusarinine C:proton symporter activity [GO:0015346] (molecular function) Also known as: ferric triacetylfusarinine C:hydrogen symporter activity Sources: TC:2.A.1.16.3 Relationships: is a type of solute:proton symporter activity [GO:0015295]; is_a siderophore-iron transmembrane transporter activity [GO:0015343]; is a type of ferric triacetylfusarinine C transmembrane transporter activity [GO:0015621]; is part of GO:0015686 Definition: Enables the transfer of a solute or solutes from one side of a membrane to the other according to the reaction: ferric triacetylfusarinine C(out) + H+(out) = ferric triacetylfusarinine C(in) + H+(in).